chemokine activity [GO:0008009] (molecular function) Definition: The function of a family of small chemotactic cytokines; their name is derived from their ability to induce directed chemotaxis in nearby responsive cells. All chemokines possess a number of conserved cysteine residues involved in intramolecular disulfide bond formation. Some chemokines are considered pro-inflammatory and can be induced during an immune response to recruit cells of the immune system to a site of infection, while others are considered homeostatic and are involved in controlling the migration of cells during normal processes of tissue maintenance or development. Chemokines are found in all vertebrates, some viruses and some bacteria. References: PMID:12183377 Sources: GOC:BHF, GOC:rl, Wikipedia:Chemokine Relationships: is a type of cytokine activity [GO:0005125]; is a type of GO:0042379; is part of cell chemotaxis [GO:0060326] Regulation: regulated by GO:1900136; negatively regulated by negative regulation of chemokine activity [GO:1900137]